negative regulation of cardiac muscle cell differentiation [GO:2000726] (biological process) Subtypes: GO:1905305 Also known as: negative regulation of cardiomyocyte differentiation, negative regulation of heart muscle cell differentiation Relationships: is a type of GO:0051154; is_a negative regulation of cardiocyte differentiation [GO:1905208]; is a type of GO:2000725; negatively regulates cardiac muscle cell differentiation [GO:0055007] Sources: GOC:BHF Definition: Any process that stops, prevents or reduces the frequency, rate or extent of cardiac muscle cell differentiation.